{
  "gene_name": "Homeobox protein GBX-2",
  "gene": "UniProtKB:P52951",
  "gene_symbol": "GBX2",
  "term_label": "regulation of transcription by RNA polymerase II",
  "term_id": "GO:0006357"
}